{
  "term_id": "GO:0006357",
  "gene_name": "Transcription factor Sp3",
  "term_label": "regulation of transcription by RNA polymerase II",
  "gene_symbol": "SP3",
  "gene": "UniProtKB:Q02447"
}